negative regulation of integrin-mediated signaling pathway [GO:2001045] (biological process) Definition: Any process that stops, prevents or reduces the frequency, rate or extent of integrin-mediated signaling pathway. Sources: GOC:obol Also known as: negative regulation of integrin-mediated signalling pathway Relationships: is a type of negative regulation of signal transduction [GO:0009968]; is a type of regulation of integrin-mediated signaling pathway [GO:2001044]; negatively regulates GO:0007229